{
  "gene_name": "Cysteine-rich tail protein 1",
  "gene_symbol": "CYSRT1",
  "term_id": "UNKNOWN:0002",
  "gene": "UniProtKB:A8MQ03",
  "term_label": "Unknown biological process"
}